guanosine-3',5'-bis(diphosphate) 3'-diphosphatase activity [GO:0008893] (MF) Also known as: guanosine-3',5'-bis(diphosphate) 3'-diphosphohydrolase activity, guanosine-3',5'-bis(diphosphate) 3'-pyrophosphohydrolase activity, (ppGpp)ase activity, PpGpp phosphohydrolase activity, PpGpp-3'-pyrophosphohydrolase activity, guanosine-3',5'-bis(diphosphate) 3'-pyrophosphatase activity, penta-phosphate guanosine-3'-diphosphohydrolase activity, penta-phosphate guanosine-3'-pyrophosphohydrolase activity Sources: RHEA:14253 Definition: Catalysis of the reaction: guanosine 3',5'-bis(diphosphate) + H2O = diphosphate + GDP + H+. Relationships: is a type of GO:0016794